polymyxin transport [GO:0042893] (biological process) Definition: The directed movement of polymyxin, any of a group of related antibiotics produced by Bacillus polymyxa and active against most Gram-negative bacteria, into, out of or within a cell, or between cells, by means of some agent such as a transporter or pore. Relationships: is_a lipid transport [GO:0006869]; is a type of amide transport [GO:0042886] Sources: GOC:jl